emodin biosynthetic process [GO:1900575] (biological process) Definition: The chemical reactions and pathways resulting in the formation of emodin. Sources: GOC:TermGenie, GOC:di Also known as: emodin anabolism, emodin biosynthesis, emodin formation, emodin synthesis Relationships: is a type of GO:0042181; is a type of secondary metabolite biosynthetic process [GO:0044550]; is_a phenol-containing compound biosynthetic process [GO:0046189] Regulation: regulated by regulation of emodin biosynthetic process [GO:1900664]; negatively regulated by negative regulation of emodin biosynthetic process [GO:1900665]; positively regulated by positive regulation of emodin biosynthetic process [GO:1900666]